{
  "term_label": "cell chemotaxis",
  "gene_symbol": "XCL1",
  "gene_name": "Lymphotactin",
  "gene": "UniProtKB:P47992",
  "term_id": "GO:0060326"
}